{
  "gene_name": "Signal-regulatory protein delta",
  "term_id": "GO:0005886",
  "gene": "UniProtKB:Q9H106",
  "term_label": "plasma membrane",
  "gene_symbol": "SIRPD"
}